{
  "gene": "UniProtKB:Q5T5A8",
  "gene_symbol": "LCE3C",
  "gene_name": "Late cornified envelope protein 3C",
  "term_id": "UNKNOWN:0001",
  "term_label": "Unknown molecular function"
}